{
  "term_id": "GO:0019373",
  "gene_name": "Cytochrome P450 2A6",
  "gene_symbol": "CYP2A6",
  "term_label": "epoxygenase P450 pathway",
  "gene": "UniProtKB:P11509"
}